{
  "gene_symbol": "SIGLEC8",
  "term_id": "GO:0007155",
  "gene": "UniProtKB:Q9NYZ4",
  "term_label": "cell adhesion",
  "gene_name": "Sialic acid-binding Ig-like lectin 8"
}